{
  "gene_symbol": "TEAD2",
  "gene_name": "Transcriptional enhancer factor TEF-4",
  "term_id": "GO:0035329",
  "term_label": "hippo signaling",
  "gene": "UniProtKB:Q15562"
}